response to prostaglandin E [GO:0034695] (biological process) Subtypes: cellular response to prostaglandin E stimulus [GO:0071380] Also known as: response to prostaglandin E stimulus Relationships: is a type of response to prostaglandin [GO:0034694]; is a type of response to alcohol [GO:0097305]; is a type of response to ketone [GO:1901654] Sources: GOC:BHF, GOC:vk Definition: Any process that results in a change in state or activity of a cell or an organism (in terms of movement, secretion, enzyme production, gene expression, etc.) as a result of a prostagladin E stimulus.